{
  "term_label": "cilium assembly",
  "gene_name": "F-box_WD repeat-containing protein 8",
  "gene_symbol": "FBXW8",
  "gene": "UniProtKB:Q8N3Y1",
  "term_id": "GO:0060271"
}